{
  "term_id": "GO:0007186",
  "term_label": "G protein-coupled receptor signaling pathway",
  "gene_symbol": "ADGRL3",
  "gene": "UniProtKB:Q9HAR2",
  "gene_name": "Adhesion G protein-coupled receptor L3"
}